positive regulation of gastric acid secretion [GO:0060454] (biological process) Sources: GOC:dph, GOC:tb Definition: Any process that increases the rate frequency or extent of gastric secretion. Gastric secretion is the regulated release of gastric acid (hydrochloric acid) by parietal or oxyntic cells during digestion. Subtypes: GO:1903641 Relationships: is_a positive regulation of secretion [GO:0051047]; is a type of regulation of gastric acid secretion [GO:0060453]; is a type of positive regulation of digestive system process [GO:0060456]; positively regulates gastric acid secretion [GO:0001696]